peptidyl-serine O-acetylation [GO:0030919] (biological process) Definition: The acetylation of peptidyl-serine to form peptidyl-O-acetyl-L-serine. References: PMID:489587, PMID:7309355 Sources: RESID:AA0364 Relationships: is a type of peptidyl-serine modification [GO:0018209]; is a type of peptidyl-serine acetylation [GO:0030920]